{
  "gene_symbol": "TMEM183BP",
  "gene": "UniProtKB:Q1AE95",
  "term_id": "GO:0019005",
  "term_label": "SCF ubiquitin ligase complex",
  "gene_name": "Putative transmembrane protein 183BP"
}